{
  "gene_name": "Uncharacterized protein C1orf127",
  "gene_symbol": "C1orf127",
  "term_label": "Unknown biological process",
  "term_id": "UNKNOWN:0002",
  "gene": "UniProtKB:Q8N9H9"
}